{
  "gene_symbol": "NFE2L1",
  "gene": "UniProtKB:Q14494",
  "term_id": "GO:0006357",
  "gene_name": "Endoplasmic reticulum membrane sensor NFE2L1",
  "term_label": "regulation of transcription by RNA polymerase II"
}